mitochondrial respiratory chain complex III assembly [GO:0034551] (biological process) Relationships: is a type of respiratory chain complex III assembly [GO:0017062]; is a type of mitochondrial respiratory chain complex assembly [GO:0033108] Sources: GOC:dgf, GOC:mcc Also known as: mitochondrial cytochrome bc(1) complex assembly Definition: The aggregation, arrangement and bonding together of a set of components to form the cytochrome bc(1) complex (also known as ubiquinol-cytochrome c reductase), in the mitochondrial inner membrane.